negative regulation of photosynthesis [GO:1905156] (biological process) Definition: Any process that stops, prevents or reduces the frequency, rate or extent of photosynthesis. References: PMID:7592491 Sources: GOC:TermGenie, GO_REF:0000058 Also known as: down regulation of photosynthesis, down-regulation of photosynthesis, downregulation of photosynthesis, inhibition of photosynthesis Relationships: is_a negative regulation of metabolic process [GO:0009892]; is a type of GO:0010109; negatively regulates photosynthesis [GO:0015979] Subtypes: negative regulation of photosynthesis, light reaction [GO:0043155], negative regulation of reductive pentose-phosphate cycle [GO:0080153]